{
  "gene_name": "Acetyl-coenzyme A synthetase 2-like, mitochondrial",
  "term_id": "GO:0003987",
  "term_label": "acetate-CoA ligase activity",
  "gene_symbol": "ACSS1",
  "gene": "UniProtKB:Q9NUB1"
}